regulation of auxin biosynthetic process [GO:0010600] (biological process) Subtypes: positive regulation of auxin biosynthetic process [GO:0010601], regulation of indoleacetic acid biosynthetic process via tryptophan [GO:1901996] References: PMID:18287041 Definition: Any process that modulates the frequency, rate or extent of the chemical reactions and pathways resulting in the formation of auxins, plant hormones that regulate aspects of plant growth. Relationships: is a type of regulation of hormone biosynthetic process [GO:0046885]; is a type of regulation of auxin metabolic process [GO:0090354]; RO_0002211 GO:0009851